{
  "term_id": "UNKNOWN:0001",
  "gene_symbol": "C1QTNF5",
  "gene": "UniProtKB:Q9BXJ0",
  "term_label": "Unknown molecular function",
  "gene_name": "Complement C1q tumor necrosis factor-related protein 5"
}